B cell receptor apoptotic signaling pathway [GO:1990117] (biological process) Relationships: is a type of B cell receptor signaling pathway [GO:0050853]; is a type of GO:0097191; is part of B cell apoptotic process [GO:0001783] References: PMID:15214043 Sources: GOC:BHF, GOC:mtg_apoptosis, GOC:rl Definition: An extrinsic apoptotic signaling pathway initiated by the cross-linking of an antigen receptor on a B cell. Also known as: B cell receptor extrinsic apoptotic signaling pathway, extrinsic apoptotic signaling pathway via B cell antigen receptor, extrinsic apoptotic signaling pathway via BCR